{
  "gene": "UniProtKB:P20671",
  "gene_name": "Histone H2A type 1-D",
  "gene_symbol": "H2AC7",
  "term_label": "nucleus",
  "term_id": "GO:0005634"
}